phosphatidylinositol-3,5-bisphosphate binding [GO:0080025] (molecular function) Definition: Binding to phosphatidylinositol-3,5-bisphosphate, a derivative of phosphatidylinositol in which the inositol ring is phosphorylated at the 3' and 5' positions. References: PMID:18397324 Sources: GOC:bf Relationships: is_a anion binding [GO:0043168]; is a type of phosphatidylinositol bisphosphate binding [GO:1902936] Also known as: PtdIns(3,5)P2 binding